protocadherin-alpha-v4-protocadherin-gamma-a1 complex [GO:0071184] (cellular component) References: PMID:15347688 Relationships: is a type of protocadherin-alpha-protocadherin-gamma complex [GO:0071183] Also known as: Pcdhga1-Pcdha4 complex Definition: A protein complex that contains the cell adhesion molecules protocadherin-alpha-v4 and protocadherin-gamma-a1, and is involved in the regulation of protein localization to the plasma membrane.